long-chain-alcohol O-fatty-acyltransferase activity [GO:0047196] (molecular function) Definition: Catalysis of the reaction: a long-chain-alcohol + acyl-CoA = a long-chain ester + CoA. Relationships: is a type of O-acyltransferase activity [GO:0008374] Sources: EC:2.3.1.75, MetaCyc:2.3.1.75-RXN Also known as: wax ester synthase activity, acyl-CoA:long-chain-alcohol O-acyltransferase activity, wax synthase activity, wax-ester synthase activity